{
  "term_label": "cytoplasmic stress granule",
  "term_id": "GO:0010494",
  "gene_name": "Polyadenylate-binding protein 4",
  "gene_symbol": "PABPC4",
  "gene": "UniProtKB:Q13310"
}